{
  "gene_symbol": "MMP11",
  "term_label": "extracellular space",
  "gene": "UniProtKB:P24347",
  "term_id": "GO:0005615",
  "gene_name": "Stromelysin-3"
}